{
  "gene_symbol": "IKBKB",
  "term_id": "GO:0043123",
  "gene_name": "Inhibitor of nuclear factor kappa-B kinase subunit beta",
  "gene": "UniProtKB:O14920",
  "term_label": "positive regulation of canonical NF-kappaB signal transduction"
}